{
  "gene": "UniProtKB:P14625",
  "gene_name": "Endoplasmin",
  "term_label": "ATP hydrolysis activity",
  "gene_symbol": "HSP90B1",
  "term_id": "GO:0016887"
}